fatty acid peroxidase activity [GO:0047888] (molecular function) Also known as: fatty-acid peroxidase activity, hexadecanoate:hydrogen-peroxide oxidoreductase activity, long chain fatty acid peroxidase activity Definition: Catalysis of the reaction: 2 H2O2 + H+ + palmitate = CO2 + 3 H2O + pentadecanal. Sources: EC:1.11.1.3, RHEA:23960 Relationships: is a type of peroxidase activity [GO:0004601]